{
  "term_label": "pericentric heterochromatin",
  "gene": "UniProtKB:P46100",
  "term_id": "GO:0005721",
  "gene_symbol": "ATRX",
  "gene_name": "Transcriptional regulator ATRX"
}